{
  "term_label": "insulin receptor signaling pathway",
  "gene": "UniProtKB:Q16654",
  "gene_name": "[Pyruvate dehydrogenase (acetyl-transferring)] kinase isozyme 4, mitochondrial",
  "gene_symbol": "PDK4",
  "term_id": "GO:0008286"
}